{
  "term_label": "lipid binding",
  "gene_symbol": "COQ9",
  "gene_name": "Ubiquinone biosynthesis protein COQ9, mitochondrial",
  "gene": "UniProtKB:O75208",
  "term_id": "GO:0008289"
}